tryptophan N-monooxygenase activity [GO:0090489] (MF) Also known as: L-tryptophan,NADPH:oxygen oxidoreductase (N-hydroxylating, decarboxylating), tryptophan N-hydroxylase activity Relationships: is a type of oxidoreductase activity, acting on paired donors, with incorporation or reduction of molecular oxygen, reduced flavin or flavoprotein as one donor, and incorporation of one atom of oxygen [GO:0016712] Sources: RHEA:33279 Definition: Catalyzes the multi-step reaction: L-tryptophan + 2 O2 + 2 reduced [NADPH--hemoprotein reductase] = (E)-(indol-3-yl)acetaldehyde oxime + CO2 + 2 H+ + 3 H2O + 2 oxidized [NADPH--hemoprotein reductase].